{
  "gene_symbol": "GPAT2",
  "gene": "UniProtKB:Q6NUI2",
  "term_id": "GO:0006650",
  "gene_name": "Glycerol-3-phosphate acyltransferase 2, mitochondrial",
  "term_label": "glycerophospholipid metabolic process"
}